regulation of osteoclast development [GO:2001204] (biological process) Also known as: regulation of osteoclast cell development Subtypes: negative regulation of osteoclast development [GO:2001205], GO:2001206 Relationships: is a type of regulation of hemopoiesis [GO:1903706]; regulates osteoclast development [GO:0036035] Definition: Any process that modulates the frequency, rate or extent of osteoclast development. Sources: GOC:obol